{
  "gene_name": "Autophagy-related protein 9A",
  "gene_symbol": "ATG9A",
  "gene": "UniProtKB:Q7Z3C6",
  "term_label": "phagophore assembly site",
  "term_id": "GO:0000407"
}